{
  "gene_name": "Eukaryotic translation initiation factor 1",
  "term_id": "UNKNOWN:0002",
  "term_label": "Unknown biological process",
  "gene": "UniProtKB:P41567",
  "gene_symbol": "EIF1"
}